{
  "term_label": "cytoplasm",
  "gene": "UniProtKB:Q9C098",
  "term_id": "GO:0005737",
  "gene_symbol": "DCLK3",
  "gene_name": "Serine_threonine-protein kinase DCLK3"
}